mitochondrial srRNA export from mitochondrion [GO:0019092] (biological process) Definition: The process in which a srRNA, small subunit ribosomal ribonucleic acid, is transported from the mitochondrial matrix into the cytosol. Sources: GOC:ai Relationships: is a type of mitochondrial rRNA export from mitochondrion [GO:0019090] Also known as: export of mitochondrial srRNA, mitochondrial srRNA export, mitochondrial srRNA export from mitochondria, mitochondrial srRNA export out of mitochondrion, mitochondrial srRNA transport from mitochondrion, mitochondrial srRNA, mitochondrial export